{
  "gene": "UniProtKB:O76036",
  "term_id": "GO:0004888",
  "gene_name": "Natural cytotoxicity triggering receptor 1",
  "gene_symbol": "NCR1",
  "term_label": "transmembrane signaling receptor activity"
}